{
  "gene_symbol": "POU6F1",
  "term_label": "DNA-binding transcription factor activity, RNA polymerase II-specific",
  "gene_name": "POU domain, class 6, transcription factor 1",
  "gene": "UniProtKB:Q14863",
  "term_id": "GO:0000981"
}